{
  "gene_symbol": "PRKCZ",
  "term_id": "GO:0035556",
  "term_label": "intracellular signal transduction",
  "gene_name": "Protein kinase C zeta type",
  "gene": "UniProtKB:Q05513"
}